{
  "gene_symbol": "ASTN1",
  "term_label": "Unknown molecular function",
  "term_id": "UNKNOWN:0001",
  "gene": "UniProtKB:O14525",
  "gene_name": "Astrotactin-1"
}